{
  "gene_name": "D-dopachrome decarboxylase-like protein",
  "term_id": "GO:0005615",
  "term_label": "extracellular space",
  "gene": "UniProtKB:A6NHG4",
  "gene_symbol": "DDTL"
}